{
  "term_id": "GO:0042105",
  "gene": "UniProtKB:P07766",
  "gene_symbol": "CD3E",
  "gene_name": "T-cell surface glycoprotein CD3 epsilon chain",
  "term_label": "alpha-beta T cell receptor complex"
}